P-body [GO:0000932] (cellular component) References: PMID:12730603 Sources: GOC:clt Relationships: is_a cytoplasmic ribonucleoprotein granule [GO:0036464] Definition: A focus in the cytoplasm where mRNAs may become inactivated by decapping or some other mechanism. Protein and RNA localized to these foci are involved in mRNA degradation, nonsense-mediated mRNA decay (NMD), translational repression, and RNA-mediated gene silencing. Also known as: P body, cytoplasmic mRNA processing body, cytoplasmic foci